regulation of backward locomotion [GO:0043058] (biological process) Sources: GOC:go_curators Definition: Any process that modulates the speed, mechanical force, or rhythm of the posterior movement of an organism. Subtypes: GO:1905851, positive regulation of backward locomotion [GO:1905852] Relationships: is a type of regulation of locomotion [GO:0040012]; regulates backward locomotion [GO:0043057]